{
  "gene_name": "Large ribosomal subunit protein eL29",
  "term_label": "cytoplasmic translation",
  "term_id": "GO:0002181",
  "gene_symbol": "RPL29",
  "gene": "UniProtKB:P47914"
}